{
  "term_label": "dendrite self-avoidance",
  "gene_name": "Basigin",
  "term_id": "GO:0070593",
  "gene": "UniProtKB:P35613",
  "gene_symbol": "BSG"
}